negative regulation of NAD metabolic process [GO:1902689] (biological process) Definition: Any process that stops, prevents or reduces the frequency, rate or extent of NAD metabolic process. References: PMID:19846558 Sources: GOC:TermGenie, GOC:di, GO_REF:0000058 Also known as: down regulation of NAD (oxidized) metabolic process, down regulation of NAD (oxidized) metabolism, down regulation of NAD metabolic process, down regulation of NAD metabolism, down regulation of nicotinamide adenine dinucleotide metabolic process, down regulation of nicotinamide adenine dinucleotide metabolism, down regulation of oxidized NAD metabolic process, down regulation of oxidized NAD metabolism, down regulation of oxidized nicotinamide adenine dinucleotide metabolic process, down regulation of oxidized nicotinamide adenine dinucleotide metabolism, down-regulation of NAD (oxidized) metabolic process, down-regulation of NAD (oxidized) metabolism, down-regulation of NAD metabolic process, down-regulation of NAD metabolism, down-regulation of nicotinamide adenine dinucleotide metabolic process, down-regulation of nicotinamide adenine dinucleotide metabolism, down-regulation of oxidized NAD metabolic process, down-regulation of oxidized NAD metabolism, down-regulation of oxidized nicotinamide adenine dinucleotide metabolic process, down-regulation of oxidized nicotinamide adenine dinucleotide metabolism, downregulation of NAD (oxidized) metabolic process, downregulation of NAD (oxidized) metabolism, downregulation of NAD metabolic process, downregulation of NAD metabolism, downregulation of nicotinamide adenine dinucleotide metabolic process, downregulation of nicotinamide adenine dinucleotide metabolism, downregulation of oxidized NAD metabolic process, downregulation of oxidized NAD metabolism, downregulation of oxidized nicotinamide adenine dinucleotide metabolic process, downregulation of oxidized nicotinamide adenine dinucleotide metabolism, negative regulation of NAD (oxidized) metabolic process, negative regulation of NAD (oxidized) metabolism, negative regulation of NAD metabolism, negative regulation of nicotinamide adenine dinucleotide metabolic process, negative regulation of nicotinamide adenine dinucleotide metabolism, negative regulation of oxidized NAD metabolic process, negative regulation of oxidized NAD metabolism, negative regulation of oxidized nicotinamide adenine dinucleotide metabolic process, negative regulation of oxidized nicotinamide adenine dinucleotide metabolism, down regulation of NAD phosphorylation and dephosphorylation, down-regulation of NAD phosphorylation and dephosphorylation, downregulation of NAD phosphorylation and dephosphorylation, inhibition of NAD (oxidized) metabolic process, inhibition of NAD (oxidized) metabolism, inhibition of NAD metabolic process, inhibition of NAD metabolism, inhibition of NAD phosphorylation and dephosphorylation, inhibition of nicotinamide adenine dinucleotide metabolic process, inhibition of nicotinamide adenine dinucleotide metabolism, inhibition of oxidized NAD metabolic process, inhibition of oxidized NAD metabolism, inhibition of oxidized nicotinamide adenine dinucleotide metabolic process, inhibition of oxidized nicotinamide adenine dinucleotide metabolism, negative regulation of NAD phosphorylation and dephosphorylation Relationships: is a type of negative regulation of purine nucleotide metabolic process [GO:1900543]; is a type of regulation of NAD metabolic process [GO:1902688]; negatively regulates NAD+ metabolic process [GO:0019674] Subtypes: negative regulation of 'de novo' NAD biosynthetic process from L-tryptophan [GO:1905013]